structural constituent of chromatin [GO:0030527] (molecular function) Sources: GOC:ai Definition: The action of a molecule that contributes to the structural integrity of chromatin. Relationships: is a type of structural molecule activity [GO:0005198]; occurs in GO:0000785